{
  "term_label": "chromatin organization",
  "gene_name": "Calcineurin-binding protein cabin-1",
  "term_id": "GO:0006325",
  "gene_symbol": "CABIN1",
  "gene": "UniProtKB:Q9Y6J0"
}